{
  "gene_symbol": "AIF1",
  "term_id": "GO:0097178",
  "term_label": "ruffle assembly",
  "gene_name": "Allograft inflammatory factor 1",
  "gene": "UniProtKB:P55008"
}